{
  "term_id": "UNKNOWN:0001",
  "gene_symbol": "WDR88",
  "gene": "UniProtKB:Q6ZMY6",
  "gene_name": "WD repeat-containing protein 88",
  "term_label": "Unknown molecular function"
}